gas transport [GO:0015669] (biological process) Sources: GOC:ai Definition: The directed movement of substances that are gaseous in normal living conditions into, out of or within a cell, or between cells, by means of some agent such as a transporter or pore. Subtypes: GO:0015670, oxygen transport [GO:0015671] Relationships: is_a transport [GO:0006810]